{
  "term_id": "GO:0003712",
  "term_label": "transcription coregulator activity",
  "gene": "UniProtKB:O94983",
  "gene_name": "Calmodulin-binding transcription activator 2",
  "gene_symbol": "CAMTA2"
}